{
  "term_label": "protein-RNA adaptor activity",
  "gene": "UniProtKB:Q01085",
  "gene_symbol": "TIAL1",
  "gene_name": "Nucleolysin TIAR",
  "term_id": "GO:0140517"
}